{
  "term_label": "serine-type endopeptidase activity",
  "gene": "UniProtKB:Q2T9J0",
  "gene_symbol": "TYSND1",
  "gene_name": "Peroxisomal leader peptide-processing protease",
  "term_id": "GO:0004252"
}